{
  "term_id": "GO:0035663",
  "gene_name": "Toll-like receptor 1",
  "gene": "UniProtKB:Q15399",
  "term_label": "Toll-like receptor 2 binding",
  "gene_symbol": "TLR1"
}